{
  "term_label": "signal transduction",
  "term_id": "GO:0007165",
  "gene_symbol": "CBLC",
  "gene_name": "E3 ubiquitin-protein ligase CBL-C",
  "gene": "UniProtKB:Q9ULV8"
}